oviduct epithelium development [GO:0035846] (biological process) Definition: The progression of the oviduct epithelium over time from its initial formation to the mature structure. An oviduct is a tube through which an ova passes from the ovary to the uterus, or from the ovary to the outside of the organism. The oviduct epithelium is the specialized epithelium that lines the oviduct. References: PMID:34496237 Sources: GOC:yaf Also known as: fallopian tube epithelium development Relationships: is a type of developmental process involved in reproduction [GO:0003006]; is a type of epithelium development [GO:0060429]; is part of oviduct development [GO:0060066] Subtypes: uterine epithelium development [GO:0035847]